{
  "term_id": "UNKNOWN:0003",
  "gene_symbol": "SPATA1",
  "term_label": "Unknown cellular component",
  "gene_name": "Spermatogenesis-associated protein 1",
  "gene": "UniProtKB:Q5VX52"
}